{
  "term_label": "olfactory receptor activity",
  "term_id": "GO:0004984",
  "gene_symbol": "OR10AC1",
  "gene": "UniProtKB:Q8NH08",
  "gene_name": "Olfactory receptor 10AC1"
}